{
  "term_id": "UNKNOWN:0003",
  "gene_name": "Zinc finger protein 287",
  "gene": "UniProtKB:Q9HBT7",
  "gene_symbol": "ZNF287",
  "term_label": "Unknown cellular component"
}